{
  "term_id": "GO:0005886",
  "gene_symbol": "NT5E",
  "gene": "UniProtKB:P21589",
  "gene_name": "5'-nucleotidase",
  "term_label": "plasma membrane"
}